{
  "gene_symbol": "ZNF446",
  "term_id": "GO:0006357",
  "gene": "UniProtKB:Q9NWS9",
  "gene_name": "Zinc finger protein 446",
  "term_label": "regulation of transcription by RNA polymerase II"
}